{
  "gene": "UniProtKB:P62955",
  "term_label": "channel regulator activity",
  "gene_symbol": "CACNG7",
  "gene_name": "Voltage-dependent calcium channel gamma-7 subunit",
  "term_id": "GO:0016247"
}